{
  "gene_symbol": "IDS",
  "term_id": "UNKNOWN:0002",
  "gene_name": "Iduronate 2-sulfatase",
  "term_label": "Unknown biological process",
  "gene": "UniProtKB:P22304"
}